aromatic amino acid family catabolic process to alcohol via Ehrlich pathway [GO:0000949] (biological process) Definition: The chemical reactions and pathways involving the catabolism of aromatic amino acids to produce aromatic alcohols with one carbon less than the starting amino acid. In S. cerevisiae, this is known to occur for leucine, isoleucine, valine, methionine, phenylalanine, tyrosine, or tryptophan. When an aromatic family amino acid, phenylalanine, tyrosine, or tryptophan, is used as the substrate, 2-phenylethanol, 4-hydroxyphenylethanol, or tryptophol, respectively, is produced. Often referred to as the Ehrlich pathway, these reactions generally occur during fermentation to produce a variety of alcohols, often collectively referred to as fusel alcohols. Depending on the redox state of the cells, carboxylic acid derivatives may be produced instead of alcohols. References: PMID:18281432 Sources: GOC:krc Relationships: is a type of amino acid catabolic process to alcohol via Ehrlich pathway [GO:0000947]; is a type of aromatic amino acid family catabolic process [GO:0009074]